{
  "term_id": "GO:0006401",
  "gene_symbol": "RNASET2",
  "term_label": "RNA catabolic process",
  "gene_name": "Ribonuclease T2",
  "gene": "UniProtKB:O00584"
}